aminotriazole transmembrane transporter activity [GO:1901478] (molecular function) Definition: Enables the transfer of amitrole from one side of a membrane to the other. Relationships: is a type of azole transmembrane transporter activity [GO:1901474] Also known as: aminotriazole transporter activity Subtypes: aminotriazole:proton antiporter activity [GO:0015314] Sources: GOC:TermGenie